{
  "gene_name": "Transmembrane protein 128",
  "gene": "UniProtKB:Q5BJH2",
  "gene_symbol": "TMEM128",
  "term_label": "Unknown molecular function",
  "term_id": "UNKNOWN:0001"
}